{
  "gene": "UniProtKB:O75832",
  "gene_name": "26S proteasome non-ATPase regulatory subunit 10",
  "term_id": "GO:0005856",
  "term_label": "cytoskeleton",
  "gene_symbol": "PSMD10"
}